cognition [GO:0050890] (biological process) Sources: ISBN:0721619908 Subtypes: learning or memory [GO:0007611], sensory processing [GO:0050893] Definition: The operation of the mind by which an organism becomes aware of objects of thought or perception; it includes the mental activities associated with thinking, learning, and memory. Relationships: is a type of GO:0050877